actin-myosin filament sliding [GO:0033275] (biological process) Also known as: actin filament sliding Subtypes: GO:0030049 Definition: The sliding movement of actin thin filaments and myosin thick filaments past each other. Relationships: is a type of actin-mediated cell contraction [GO:0070252] Sources: GOC:pf